{
  "gene": "UniProtKB:Q96LW4",
  "gene_symbol": "PRIMPOL",
  "term_label": "chromatin binding",
  "gene_name": "DNA-directed primase_polymerase protein",
  "term_id": "GO:0003682"
}